{
  "gene_name": "Neuroendocrine convertase 1",
  "term_id": "GO:0005615",
  "term_label": "extracellular space",
  "gene": "UniProtKB:P29120",
  "gene_symbol": "PCSK1"
}